{
  "gene_symbol": "COQ2",
  "term_label": "4-hydroxybenzoate polyprenyltransferase activity",
  "term_id": "GO:0008412",
  "gene_name": "4-hydroxybenzoate polyprenyltransferase, mitochondrial",
  "gene": "UniProtKB:Q96H96"
}